{
  "gene": "UniProtKB:Q68CR1",
  "term_id": "UNKNOWN:0003",
  "gene_name": "Protein sel-1 homolog 3",
  "gene_symbol": "SEL1L3",
  "term_label": "Unknown cellular component"
}